{
  "term_label": "Cul2-RING ubiquitin ligase complex",
  "gene_symbol": "ZSWIM5",
  "term_id": "GO:0031462",
  "gene_name": "Zinc finger SWIM domain-containing protein 5",
  "gene": "UniProtKB:Q9P217"
}